{
  "gene_symbol": "RCVRN",
  "gene_name": "Recoverin",
  "gene": "UniProtKB:P35243",
  "term_label": "calcium ion binding",
  "term_id": "GO:0005509"
}